synapse [GO:0045202] (cellular component) Subtypes: neuromuscular junction [GO:0031594], excitatory synapse [GO:0060076], GO:0060077, GO:0097470, Schaffer collateral - CA1 synapse [GO:0098685], GO:0098690, dopaminergic synapse [GO:0098691], noradrenergic synapse [GO:0098692], glutamatergic synapse [GO:0098978], polyadic synapse [GO:0098979], GO:0098981, GABA-ergic synapse [GO:0098982], neuron to neuron synapse [GO:0098984], GO:0099154, cerebellar Golgi cell to granule cell synapse [GO:0099192], GO:0140240 References: PMID:24619342, PMID:29383328, PMID:31998110 Sources: GOC:aruk, ISBN:0198506732 Also known as: synaptic junction, mixed synapse, electrotonic synapse Relationships: is a type of cell junction [GO:0030054] Definition: The junction between an axon of one neuron and a dendrite of another neuron, a muscle fiber or a glial cell. As the axon approaches the synapse it enlarges into a specialized structure, the presynaptic terminal bouton, which contains mitochondria and synaptic vesicles. At the tip of the terminal bouton is the presynaptic membrane; facing it, and separated from it by a minute cleft (the synaptic cleft) is a specialized area of membrane on the receiving cell, known as the postsynaptic membrane. In response to the arrival of nerve impulses, the presynaptic terminal bouton secretes molecules of neurotransmitters into the synaptic cleft. These diffuse across the cleft and transmit the signal to the postsynaptic membrane.